gene conversion of immunoglobulin genes [GO:0002206] (biological process) Relationships: is a type of GO:0002565; is a type of somatic diversification of immunoglobulins [GO:0016445]; is a type of gene conversion [GO:0035822] References: PMID:14991701 Sources: GOC:add Also known as: gene conversion of antibody genes Subtypes: gene conversion of immunoglobulin genes involved in immune response [GO:0002207] Definition: The somatic process in which immunoglobulin genes are diversified through the mechanism of gene conversion.